{
  "gene_symbol": "FOXL3",
  "gene_name": "Forkhead box protein L3",
  "term_id": "GO:0006357",
  "term_label": "regulation of transcription by RNA polymerase II",
  "gene": "UniProtKB:A0A1W2PRP0"
}